{
  "term_id": "GO:1902476",
  "gene": "UniProtKB:Q9H2B4",
  "gene_name": "Sulfate anion transporter 1",
  "gene_symbol": "SLC26A1",
  "term_label": "chloride transmembrane transport"
}